tight junction organization [GO:0120193] (biological process) Definition: A process that is carried out at the cellular level which results in the assembly, arrangement of constituent parts, or disassembly of a tight junction. A tight junction seals cells together in an epithelium in a way that prevents even small molecules from leaking from one side of the sheet to the other. Also known as: occluding cell junction organization, occluding junction organization Subtypes: tight junction assembly [GO:0120192], GO:1905071 Sources: GOC:krc, GOC:rl Relationships: is a type of cell-cell junction organization [GO:0045216]